mitotic DNA replication maintenance of fidelity [GO:1990505] (biological process) Definition: Any maintenance of fidelity that is involved in mitotic cell cycle DNA replication. Subtypes: mitotic recombination-dependent replication fork processing [GO:1990426] Relationships: is a type of cell cycle DNA replication maintenance of fidelity [GO:1902298]; is a type of mitotic cell cycle process [GO:1903047]; is part of mitotic DNA replication [GO:1902969] References: PMID:19185548 Also known as: maintenance of fidelity involved in mitotic DNA replication, maintenance of fidelity involved in mitotic cell cycle DNA replication